{
  "term_id": "GO:0005615",
  "gene_name": "Ribonuclease K6",
  "term_label": "extracellular space",
  "gene": "UniProtKB:Q93091",
  "gene_symbol": "RNASE6"
}